{
  "gene": "UniProtKB:Q8IVQ6",
  "gene_name": "Palmitoyltransferase ZDHHC21",
  "gene_symbol": "ZDHHC21",
  "term_id": "GO:0019706",
  "term_label": "protein-cysteine S-palmitoyltransferase activity"
}